{
  "term_id": "GO:0032760",
  "gene": "UniProtKB:P12314",
  "gene_name": "High affinity immunoglobulin gamma Fc receptor I",
  "gene_symbol": "FCGR1A",
  "term_label": "positive regulation of tumor necrosis factor production"
}